{
  "gene_symbol": "AREG",
  "term_id": "GO:0005154",
  "gene": "UniProtKB:P15514",
  "term_label": "epidermal growth factor receptor binding",
  "gene_name": "Amphiregulin"
}